dihydrochelirubine 12-monooxygenase activity [GO:0047089] (molecular function) Definition: Catalysis of the reaction: dihydrochelirubine + H+ + NADPH + O2 = 12-hydroxydihydrochelirubine + H2O + NADP+. Sources: EC:1.14.14.101, RHEA:10156 Relationships: is a type of oxidoreductase activity, acting on paired donors, with incorporation or reduction of molecular oxygen, NAD(P)H as one donor, and incorporation of one atom of oxygen [GO:0016709] Also known as: dihydrochelirubine 12-hydroxylase activity, dihydrochelirubine,NADPH:oxygen oxidoreductase (12-hydroxylating)